{
  "gene_name": "Transcobalamin-1",
  "term_id": "GO:0015889",
  "gene_symbol": "TCN1",
  "gene": "UniProtKB:P20061",
  "term_label": "cobalamin transport"
}